{
  "term_id": "GO:0005737",
  "gene_name": "Deleted in azoospermia-like",
  "gene": "UniProtKB:Q92904",
  "gene_symbol": "DAZL",
  "term_label": "cytoplasm"
}